{
  "gene": "UniProtKB:Q5H9L2",
  "gene_name": "Transcription elongation factor A protein-like 5",
  "term_id": "UNKNOWN:0002",
  "gene_symbol": "TCEAL5",
  "term_label": "Unknown biological process"
}